{
  "gene_name": "Probable non-functional immunoglobulin heavy variable 7-81",
  "term_label": "immunoglobulin mediated immune response",
  "term_id": "GO:0016064",
  "gene": "UniProtKB:A0A0B4J1V7",
  "gene_symbol": "IGHV7-81"
}